{
  "gene": "UniProtKB:O43316",
  "term_label": "regulation of transcription by RNA polymerase II",
  "term_id": "GO:0006357",
  "gene_name": "Paired box protein Pax-4",
  "gene_symbol": "PAX4"
}